tropine dehydrogenase activity [GO:0050356] (molecular function) Also known as: tropine:NADP+ 3alpha-oxidoreductase activity Definition: Catalysis of the reaction: NADP+ + tropine = H+ + NADPH + tropinone. Sources: EC:1.1.1.206, RHEA:18357 Relationships: is a type of oxidoreductase activity, acting on the CH-OH group of donors, NAD or NADP as acceptor [GO:0016616]